{
  "term_id": "UNKNOWN:0002",
  "term_label": "Unknown biological process",
  "gene_name": "Putative tyrosine-protein phosphatase TPTE",
  "gene": "UniProtKB:P56180",
  "gene_symbol": "TPTE"
}